{
  "gene": "UniProtKB:Q9UKB5",
  "term_id": "GO:0044291",
  "gene_name": "Adherens junction-associated protein 1",
  "gene_symbol": "AJAP1",
  "term_label": "cell-cell contact zone"
}